{
  "term_id": "GO:0005251",
  "term_label": "delayed rectifier potassium channel activity",
  "gene": "UniProtKB:Q9UJ90",
  "gene_symbol": "KCNE5",
  "gene_name": "Potassium voltage-gated channel subfamily E regulatory beta subunit 5"
}